{
  "term_label": "nucleus",
  "gene_name": "PSME3-interacting protein",
  "gene_symbol": "PSME3IP1",
  "gene": "UniProtKB:Q9GZU8",
  "term_id": "GO:0005634"
}